alpha-1,4-glucan glucosyltransferase (UDP-glucose donor) activity [GO:0004373] (molecular function) Also known as: glycogen (starch) synthetase activity, glyucogen (starch) synthase activity, UDP-glucose-glycogen glucosyltransferase activity, UDP-glucose:glycogen 4-alpha-D-glucosyltransferase activity, UDP-glycogen synthase activity, UDPG-glycogen synthetase activity, UDPG-glycogen transglucosylase activity, UDPglucose:glycogen 4-alpha-D-glucosyltransferase activity, uridine diphosphoglucose-glycogen glucosyltransferase activity Sources: RHEA:18549 Regulation: regulated by regulation of glycogen (starch) synthase activity [GO:2000465]; negatively regulated by negative regulation of glycogen (starch) synthase activity [GO:2000466]; positively regulated by positive regulation of glycogen (starch) synthase activity [GO:2000467] Definition: Catalysis of the reaction: [(1->4)-alpha-D-glucosyl](n) + UDP-alpha-D-glucose = [(1->4)-alpha-D-glucosyl](n+1) + H+ + UDP. Relationships: is a type of GO:0033840; is a type of UDP-glucosyltransferase activity [GO:0035251]